{
  "term_label": "heparan sulfate proteoglycan biosynthetic process",
  "gene": "UniProtKB:Q9H3R1",
  "gene_name": "Bifunctional heparan sulfate N-deacetylase_N-sulfotransferase 4",
  "term_id": "GO:0015012",
  "gene_symbol": "NDST4"
}